regulation of fumigaclavine C biosynthetic process [GO:1900837] (biological process) Definition: Any process that modulates the frequency, rate or extent of fumigaclavine C biosynthetic process. Relationships: is a type of regulation of ergot alkaloid biosynthetic process [GO:1900822]; regulates GO:1900809 Subtypes: GO:1900838, GO:1900839 Also known as: regulation of fumigaclavine C anabolism, regulation of fumigaclavine C biosynthesis, regulation of fumigaclavine C formation, regulation of fumigaclavine C synthesis Sources: GOC:TermGenie, GOC:di